sucrose:proton symporter activity [GO:0008506] (molecular function) Definition: Enables the transfer of a solute or solutes from one side of a membrane to the other according to the reaction: sucrose(out) + H+(out) = sucrose(in) + H+(in). Relationships: is a type of GO:0005351; is_a GO:0009669 Also known as: hydrogen/sucrose transporter activity, sucrose:hydrogen symporter activity Sources: TC:2.A.1.5.3